{
  "term_id": "GO:0005737",
  "term_label": "cytoplasm",
  "gene": "UniProtKB:P51812",
  "gene_symbol": "RPS6KA3",
  "gene_name": "Ribosomal protein S6 kinase alpha-3"
}